vascular endothelial growth factor production [GO:0010573] (BP) Regulation: regulated by regulation of vascular endothelial growth factor production [GO:0010574]; positively regulated by GO:0010575; negatively regulated by negative regulation of vascular endothelial growth factor production [GO:1904046] Definition: The appearance of vascular endothelial growth factor production due to biosynthesis or secretion following a cellular stimulus, resulting in an increase in its intracellular or extracellular levels. Also known as: VEGF production Relationships: is a type of GO:0001816 Sources: GOC:rl